{
  "term_label": "urea transmembrane transporter activity",
  "gene_name": "Aquaporin-9",
  "gene": "UniProtKB:O43315",
  "gene_symbol": "AQP9",
  "term_id": "GO:0015204"
}